{
  "gene": "UniProtKB:Q9H2A7",
  "gene_name": "C-X-C motif chemokine 16",
  "term_id": "GO:0008009",
  "gene_symbol": "CXCL16",
  "term_label": "chemokine activity"
}